{
  "gene_symbol": "CNOT2",
  "gene_name": "CCR4-NOT transcription complex subunit 2",
  "gene": "UniProtKB:Q9NZN8",
  "term_id": "GO:0000932",
  "term_label": "P-body"
}